NADP phosphatase activity [GO:0019178] (molecular function) Definition: Catalysis of the reaction: H2O + NADP+ = NAD+ + phosphate. Relationships: is a type of phosphatase activity [GO:0016791] Sources: RHEA:28050